wing disc anterior/posterior pattern formation [GO:0048100] (biological process) Relationships: is a type of GO:0007448; is a type of GO:0035222 References: PMID:10625531 Sources: GOC:jid Definition: The establishment, maintenance and elaboration of the anterior/posterior axis of the wing disc, a precursor to the wing.